{
  "gene": "UniProtKB:Q9NRY5",
  "gene_name": "Protein FAM114A2",
  "gene_symbol": "FAM114A2",
  "term_label": "Unknown cellular component",
  "term_id": "UNKNOWN:0003"
}